adenosylcobinamide-GDP ribazoletransferase activity [GO:0051073] (molecular function) Relationships: is a type of phosphotransferase activity, for other substituted phosphate groups [GO:0016780] Definition: Catalysis of the reaction: adenosylcobinamide-GDP + alpha-ribazole = GMP + adenosylcobalamin. Also known as: cobalamin synthase activity, CobS, adenosylcobinamide-GDP:alpha-ribazole ribazoletransferase activity, cobalamin (5'-phosphate) synthase activity, cobalamin-5'-phosphate synthase activity Sources: EC:2.7.8.26, MetaCyc:COBALAMINSYN-RXN